 [go#goslim:generic] Note: Generic GO slim